enzyme IIA-maltose transporter complex [GO:1990154] (cellular component) Also known as: EIIA(Glc)-MalFGK2 complex, EIIA(Glc)-maltose transporter complex, maltose transporter inhibitor complex Definition: A protein complex consisting of the pentameric maltose transporter complex bound to two enzyme IIA (EIIA) molecules. EIIA is a component of the glucose-specific phosphotransferase system that inhibits maltose transport from the periplasm to the cytoplasm. When EIIA-bound, the maltose transporter remains in the open, inward-facing conformation, which prevents binding of maltose-loaded maltose binding protein (MBP) to the transporter. References: PMID:23770568 Sources: GOC:bf, GOC:bhm Relationships: is a type of ATP-binding cassette (ABC) transporter complex [GO:0043190]; has part maltose transport complex [GO:1990060]